{
  "term_label": "protein N-linked glycosylation",
  "gene_name": "Alpha-1,3-mannosyl-glycoprotein 4-beta-N-acetylglucosaminyltransferase-like protein MGAT4D",
  "gene_symbol": "MGAT4D",
  "gene": "UniProtKB:A6NG13",
  "term_id": "GO:0006487"
}